{
  "gene": "UniProtKB:O75478",
  "term_id": "GO:0070461",
  "gene_symbol": "TADA2A",
  "term_label": "SAGA-type complex",
  "gene_name": "Transcriptional adapter 2-alpha"
}